{
  "term_id": "GO:0019955",
  "term_label": "cytokine binding",
  "gene": "UniProtKB:P48357",
  "gene_name": "Leptin receptor",
  "gene_symbol": "LEPR"
}